type 1 galanin receptor binding [GO:0031764] (molecular function) Sources: GOC:mah, GOC:nln Also known as: type 1 galanin receptor ligand Relationships: is a type of galanin receptor binding [GO:0031763] Definition: Binding to a type 1 galanin receptor.